{
  "gene_name": "Toll-like receptor 5",
  "gene_symbol": "TLR5",
  "term_label": "inflammatory response",
  "gene": "UniProtKB:O60602",
  "term_id": "GO:0006954"
}